{
  "gene_symbol": "CNN2",
  "term_label": "actin filament binding",
  "term_id": "GO:0051015",
  "gene_name": "Calponin-2",
  "gene": "UniProtKB:Q99439"
}